negative regulation of DNA recombinase mediator complex assembly [GO:1903873] (biological process) Definition: Any process that stops, prevents or reduces the frequency, rate or extent of DNA recombinase mediator complex assembly. References: PMID:18347097 Sources: GOC:TermGenie, GOC:rb, GO_REF:0000058 Relationships: is a type of negative regulation of protein-containing complex assembly [GO:0031333]; is a type of regulation of DNA recombinase mediator complex assembly [GO:1903872]; negatively regulates DNA recombinase mediator complex assembly [GO:1903871] Also known as: down regulation of DNA recombinase mediator complex assembly, down regulation of DNA recombinase mediator complex formation, down-regulation of DNA recombinase mediator complex assembly, down-regulation of DNA recombinase mediator complex formation, downregulation of DNA recombinase mediator complex assembly, downregulation of DNA recombinase mediator complex formation, negative regulation of DNA recombinase mediator complex formation, inhibition of DNA recombinase mediator complex assembly, inhibition of DNA recombinase mediator complex formation